regulation of mitochondrial membrane potential [GO:0051881] (biological process) Sources: GOC:ai Relationships: is a type of regulation of membrane potential [GO:0042391] Subtypes: GO:0010917, positive regulation of mitochondrial membrane potential [GO:0010918], mitochondrial depolarization [GO:0051882], regulation of mitochondrial depolarization [GO:0051900] Definition: Any process that modulates the establishment or extent of the mitochondrial membrane potential, the electric potential existing across the mitochondrial membrane arising from charges in the membrane itself and from the charges present in the media on either side of the membrane.